{
  "gene_symbol": "BTG3",
  "gene": "UniProtKB:Q14201",
  "term_label": "cytoplasm",
  "term_id": "GO:0005737",
  "gene_name": "Protein BTG3"
}